transcription regulator activity [GO:0140110] (molecular function) Subtypes: RNA-binding transcription regulator activity [GO:0001070], transcription antitermination factor activity, RNA binding [GO:0001072], transcription antitermination factor activity, DNA binding [GO:0001073], DNA-binding transcription factor activity [GO:0003700], transcription elongation factor activity [GO:0003711], GO:0003712, mitochondrial transcription factor activity [GO:0034246], anti-sigma factor antagonist activity [GO:0043856] Sources: GOC:pg, GOC:txnOH-2018, Wikipedia:Transcription_factor Relationships: is a type of molecular_function [GO:0003674] Definition: A molecular function that controls the rate, timing and/or magnitude of gene transcription. The function of transcriptional regulators is to modulate gene expression at the transcription step so that they are expressed in the right cell at the right time and in the right amount throughout the life of the cell and the organism. Genes are transcriptional units, and include bacterial operons. Regulation: RO_0002212 by transcription regulator inhibitor activity [GO:0140416]; positively regulated by transcription regulator activator activity [GO:0140537]